{
  "gene_symbol": "SMIM41",
  "term_label": "Unknown cellular component",
  "gene": "UniProtKB:A0A2R8YCJ5",
  "gene_name": "Small integral membrane protein 41",
  "term_id": "UNKNOWN:0003"
}